{
  "gene_symbol": "DLG4",
  "gene": "UniProtKB:P78352",
  "term_id": "GO:0097120",
  "term_label": "receptor localization to synapse",
  "gene_name": "Disks large homolog 4"
}